{
  "term_id": "GO:0006357",
  "gene_symbol": "ZSCAN31",
  "term_label": "regulation of transcription by RNA polymerase II",
  "gene": "UniProtKB:Q96LW9",
  "gene_name": "Zinc finger and SCAN domain-containing protein 31"
}